{
  "term_label": "positive regulation of B cell proliferation",
  "gene_name": "SAM and SH3 domain-containing protein 3",
  "gene": "UniProtKB:O75995",
  "term_id": "GO:0030890",
  "gene_symbol": "SASH3"
}